{
  "term_id": "UNKNOWN:0002",
  "term_label": "Unknown biological process",
  "gene": "UniProtKB:O95169",
  "gene_name": "NADH dehydrogenase [ubiquinone] 1 beta subcomplex subunit 8, mitochondrial",
  "gene_symbol": "NDUFB8"
}